{
  "gene": "UniProtKB:Q9H920",
  "term_label": "ERAD pathway",
  "term_id": "GO:0036503",
  "gene_symbol": "RNF121",
  "gene_name": "E3 ubiquitin ligase RNF121"
}